{
  "gene_name": "Putative olfactory receptor 2B8",
  "gene_symbol": "OR2B8",
  "term_label": "detection of chemical stimulus involved in sensory perception of smell",
  "gene": "UniProtKB:P59922",
  "term_id": "GO:0050911"
}